{
  "gene": "UniProtKB:Q6XPS3",
  "gene_name": "Phosphatidylinositol 3,4,5-trisphosphate 3-phosphatase TPTE2",
  "gene_symbol": "TPTE2",
  "term_id": "UNKNOWN:0002",
  "term_label": "Unknown biological process"
}